monoatomic cation channel activity [GO:0005261] (molecular function) Sources: GOC:def, GOC:dph, GOC:mtg_transport, GOC:pr, ISBN:0815340729 Definition: Enables the energy-independent facilitated diffusion of a monoatomic cation through a transmembrane aqueous pore or channel. Also known as: cation channel activity, cation diffusion facilitator activity, non-selective cation channel activity Regulation: positively regulated by positive regulation of cation channel activity [GO:2001259] Relationships: is a type of monoatomic ion channel activity [GO:0005216]; is a type of monoatomic cation transmembrane transporter activity [GO:0008324] Subtypes: GO:0005262, potassium channel activity [GO:0005267], GO:0005272, proton channel activity [GO:0015252], voltage-gated monoatomic cation channel activity [GO:0022843], temperature-gated cation channel activity [GO:0097604], GO:0099094, mechanosensitive monoatomic cation channel activity [GO:0140135], osmolarity-sensing monoatomic cation channel activity [GO:1990760]